positive regulation of miRNA processing [GO:1903800] (biological process) Subtypes: positive regulation of pre-miRNA processing [GO:2000633], positive regulation of primary miRNA processing [GO:2000636] Relationships: is a type of positive regulation of gene expression [GO:0010628]; is a type of regulation of miRNA processing [GO:1903798]; is a type of positive regulation of miRNA-mediated gene silencing [GO:2000637]; positively regulates miRNA processing [GO:0035196] Also known as: positive regulation of gene silencing by miRNA, production of miRNAs, positive regulation of miRNA-mediated gene silencing, production of miRNAs, positive regulation of microRNA-mediated gene silencing, production of microRNAs, positive regulation of production of microRNAs involved in gene silencing by microRNA, activation of gene silencing by miRNA, production of miRNAs, activation of miRNA processing, activation of miRNA-mediated gene silencing, production of miRNAs, activation of microRNA-mediated gene silencing, production of microRNAs, activation of production of miRNAs involved in gene silencing by miRNA, activation of production of microRNAs involved in gene silencing by microRNA, positive regulation of miRNA maturation, activation of miRNA biogenesis, activation of microRNA biogenesis, activation of microRNA biosynthesis, activation of microRNA biosynthetic process, activation of microRNA metabolic process, activation of microRNA metabolism, positive regulation of miRNA biogenesis, positive regulation of microRNA biogenesis, positive regulation of microRNA biosynthesis, positive regulation of microRNA biosynthetic process, positive regulation of microRNA metabolic process, positive regulation of microRNA metabolism, positive regulation of production of miRNAs involved in gene silencing by miRNA Definition: Any process that activates or increases the frequency, rate or extent of microRNA processing. References: PMID:22269326 Sources: GOC:BHF, GOC:BHF_miRNA, GOC:TermGenie, GOC:rph, GO_REF:0000058